{
  "gene_symbol": "CNTN5",
  "gene": "UniProtKB:O94779",
  "gene_name": "Contactin-5",
  "term_id": "GO:0030424",
  "term_label": "axon"
}